lignan metabolic process [GO:0009806] (biological process) Definition: The chemical reactions and pathways involving lignans, any member of a class of plant metabolites related to lignins. Lignans are usually found as phenylpropanoid dimers in which the phenylpropanoid units are linked tail to tail and thus having a 2,3 dibenzylbutane skeleton, but higher oligomers can also exist. Also known as: lignan metabolism Relationships: is a type of phenylpropanoid metabolic process [GO:0009698] Subtypes: lignan biosynthetic process [GO:0009807], lignan catabolic process [GO:0046273], (-)-pinoresinol metabolic process [GO:1901598], (+)-larreatricin metabolic process [GO:1901709] References: PMID:10074466 Sources: GOC:jl